{
  "gene_symbol": "PPM1D",
  "gene": "UniProtKB:O15297",
  "term_label": "negative regulation of gene expression, epigenetic",
  "term_id": "GO:0045814",
  "gene_name": "Protein phosphatase 1D"
}